{
  "gene_name": "Immunoglobulin superfamily member 1",
  "gene": "UniProtKB:Q8N6C5",
  "term_label": "plasma membrane",
  "gene_symbol": "IGSF1",
  "term_id": "GO:0005886"
}